{
  "term_id": "GO:0005886",
  "term_label": "plasma membrane",
  "gene_symbol": "STX19",
  "gene_name": "Syntaxin-19",
  "gene": "UniProtKB:Q8N4C7"
}